phosphorus-oxygen lyase activity [GO:0016849] (molecular function) Relationships: is a type of GO:0016829 Subtypes: GO:0000213, GO:0004016, guanylate cyclase activity [GO:0004383], GO:0004436, ribonuclease A activity [GO:0004522], 2-C-methyl-D-erythritol 2,4-cyclodiphosphate synthase activity [GO:0008685], Enterobacter ribonuclease activity [GO:0008847], ribonuclease T2 activity [GO:0033897], GO:0033899, rRNA endonuclease activity [GO:0033902], FAD-AMP lyase (cyclizing) activity [GO:0034012], ribonuclease T1 activity [GO:0046589], GO:0047396, cytidylate cyclase activity [GO:0047805], cyclic pyranopterin monophosphate synthase activity [GO:0061799] Definition: Catalysis of the cleavage of a phosphorus-oxygen bond by other means than by hydrolysis or oxidation, or conversely adding a group to a double bond. Sources: GOC:jl